superior olivary nucleus development [GO:0021718] (BP) Sources: GOC:cls, GOC:dgh, GOC:dph, GOC:jid, GO_REF:0000021 Definition: The process whose specific outcome is the progression of the superior olivary nucleus over time, from its formation to the mature structure. In mice, the superior olivary nucleus is a small cylindrical mass on the dorsal surface of the lateral part of the trapezoid body of the pons, and it is situated immediately above the inferior olivary nucleus. It receives projections from the cochlear nucleus and thus is involved in the perception of sound. Relationships: is a type of neural nucleus development [GO:0048857]; BFO_0000050 pons development [GO:0021548] Also known as: superior olive development